{
  "gene": "UniProtKB:Q96L11",
  "term_label": "fusion of sperm to egg plasma membrane involved in single fertilization",
  "gene_symbol": "LLCFC1",
  "term_id": "GO:0007342",
  "gene_name": "Sperm-egg fusion protein LLCFC1"
}